{
  "term_id": "UNKNOWN:0003",
  "gene": "UniProtKB:Q6UWW0",
  "term_label": "Unknown cellular component",
  "gene_name": "Lipocalin-15",
  "gene_symbol": "LCN15"
}